{
  "term_id": "GO:0042555",
  "gene": "UniProtKB:P33991",
  "gene_symbol": "MCM4",
  "gene_name": "DNA replication licensing factor MCM4",
  "term_label": "MCM complex"
}